{
  "gene_name": "Potassium_sodium hyperpolarization-activated cyclic nucleotide-gated channel 4",
  "gene": "UniProtKB:Q9Y3Q4",
  "gene_symbol": "HCN4",
  "term_label": "dendrite",
  "term_id": "GO:0030425"
}